3-hydroxybenzyl alcohol metabolic process [GO:0018921] (BP) Also known as: 3-hydroxybenzyl alcohol metabolism Relationships: is a type of alcohol metabolic process [GO:0006066]; is a type of phenol-containing compound metabolic process [GO:0018958] Sources: UM-BBD_pathwayID:mcr Definition: The chemical reactions and pathways involving 3-hydroxybenzyl alcohol, an aromatic compound which is an intermediate in several metabolic pathways, including the biosynthesis of patulin, a toxin and antiviral agent produced by some moulds such as Penicillium patulinum.